(3R)-3-hydroxyacyl-CoA dehydrogenase (NAD+) activity [GO:0106386] (MF) Definition: Catalysis of the reaction: a (3R)-3-hydroxyacyl-CoA + NAD+ = a 3-oxoacyl-CoA + NADH + H+. Relationships: is a type of oxidoreductase activity, acting on the CH-OH group of donors, NAD or NADP as acceptor [GO:0016616] Also known as: (3R)-hydroxyacyl-CoA dehydrogenase (NAD) activity, (3R)-hydroxyacyl-CoA dehydrogenase (NAD+) activity References: PMID:19571038, PMID:25203508 Sources: RHEA:32711